{
  "gene": "UniProtKB:Q58EX2",
  "gene_name": "Protein sidekick-2",
  "gene_symbol": "SDK2",
  "term_id": "GO:0045202",
  "term_label": "synapse"
}